{
  "gene_name": "Myoglobin",
  "gene": "UniProtKB:P02144",
  "term_id": "GO:0098809",
  "gene_symbol": "MB",
  "term_label": "nitrite reductase activity"
}